{
  "gene": "UniProtKB:Q8N3Z6",
  "gene_symbol": "ZCCHC7",
  "gene_name": "Zinc finger CCHC domain-containing protein 7",
  "term_label": "TRAMP complex",
  "term_id": "GO:0031499"
}